{
  "term_label": "actin binding",
  "gene_name": "Epidermal growth factor receptor kinase substrate 8-like protein 1",
  "gene": "UniProtKB:Q8TE68",
  "term_id": "GO:0003779",
  "gene_symbol": "EPS8L1"
}